{
  "term_label": "chromatin binding",
  "gene_name": "Histone acetyltransferase KAT6B",
  "gene": "UniProtKB:Q8WYB5",
  "term_id": "GO:0003682",
  "gene_symbol": "KAT6B"
}